{
  "gene_name": "Poly(ADP-ribose) glycohydrolase",
  "gene_symbol": "PARG",
  "gene": "UniProtKB:Q86W56",
  "term_label": "nucleotide-sugar metabolic process",
  "term_id": "GO:0009225"
}